plasma membrane-derived thylakoid ribulose bisphosphate carboxylase complex [GO:0048493] (cellular component) Sources: GOC:mlg, GOC:mtg_sensu Also known as: RubisCO complex, ribulose bisphosphate carboxylase complex, plasma membrane ribulose bisphosphate carboxylase complex Relationships: is a type of chromatophore ribulose bisphosphate carboxylase complex [GO:0048494]; is a type of plasma membrane protein complex [GO:0098797]; is part of bacterial thylakoid [GO:0030075] Definition: A complex, located in the plasma membrane-derived thylakoid, containing either both large and small subunits or just small subunits. It carries out the activity of producing 3-phosphoglycerate from carbon dioxide and ribulose-1,5-bisphosphate.